nucleotide receptor activity [GO:0016502] (molecular function) Subtypes: GO:0001614, G protein-coupled pyrimidinergic nucleotide receptor activity [GO:0071553] Relationships: is a type of transmembrane signaling receptor activity [GO:0004888]; has part nucleotide binding [GO:0000166] Definition: Combining with a nucleotide and transmitting the signal from one side of the membrane to the other to initiate a change in cell activity. A nucleotide is a compound that consists of a nucleoside esterified with a phosphate molecule. Sources: GOC:signaling, ISBN:0198506732